{
  "gene": "UniProtKB:Q9HCQ7",
  "term_label": "signaling receptor binding",
  "gene_symbol": "NPVF",
  "term_id": "GO:0005102",
  "gene_name": "Pro-FMRFamide-related neuropeptide VF"
}